{
  "gene_name": "Down syndrome critical region protein 9",
  "term_id": "UNKNOWN:0001",
  "gene_symbol": "DSCR9",
  "gene": "UniProtKB:P59020",
  "term_label": "Unknown molecular function"
}